regulation of cell wall macromolecule metabolic process [GO:0010981] (biological process) Definition: Any process that modulates the rate, frequency or extent of cell wall macromolecule metabolism. Cell wall macromolecule metabolic processes are the chemical reactions and pathways involving macromolecules forming, or destined to form, part of the cell wall. A cell wall is a rigid or semi-rigid envelope lying outside the cell membrane of plant, fungal and most prokaryotic cells, maintaining their shape and protecting them from osmotic lysis. Subtypes: GO:0070608, GO:0090093, regulation of cell wall (1->3)-beta-D-glucan biosynthetic process [GO:0090334], GO:2000966, regulation of plant-type cell wall cellulose biosynthetic process [GO:2001009] Sources: GOC:dph, GOC:tb Relationships: is a type of regulation of macromolecule metabolic process [GO:0060255]; regulates GO:0044036